positive regulation of cytokine production involved in immune response [GO:0002720] (biological process) Sources: GOC:add Subtypes: positive regulation of B cell cytokine production [GO:0002723], positive regulation of T cell cytokine production [GO:0002726], positive regulation of natural killer cell cytokine production [GO:0002729], positive regulation of dendritic cell cytokine production [GO:0002732], positive regulation of myeloid leukocyte cytokine production involved in immune response [GO:0061081] Also known as: activation of cytokine production during immune response, positive regulation of cytokine biosynthetic process involved in immune response, positive regulation of cytokine secretion involved in immune response, stimulation of cytokine production during immune response, positive regulation of cytokine production during immune response, up regulation of cytokine production during immune response, up-regulation of cytokine production during immune response, upregulation of cytokine production during immune response Definition: Any process that activates or increases the frequency, rate, or extent of cytokine production that contributes to an immune response. Relationships: is a type of GO:0001819; is_a positive regulation of production of molecular mediator of immune response [GO:0002702]; is a type of regulation of cytokine production involved in immune response [GO:0002718]; positively regulates GO:0002367